{
  "term_id": "GO:0005737",
  "gene": "UniProtKB:O15327",
  "gene_symbol": "INPP4B",
  "term_label": "cytoplasm",
  "gene_name": "Inositol polyphosphate 4-phosphatase type II"
}